{
  "term_id": "GO:0003714",
  "term_label": "transcription corepressor activity",
  "gene_symbol": "TLE2",
  "gene_name": "Transducin-like enhancer protein 2",
  "gene": "UniProtKB:Q04725"
}